{
  "gene_symbol": "IRS2",
  "term_label": "insulin receptor binding",
  "term_id": "GO:0005158",
  "gene": "UniProtKB:Q9Y4H2",
  "gene_name": "Insulin receptor substrate 2"
}